{
  "term_id": "GO:0004613",
  "gene": "UniProtKB:Q16822",
  "gene_symbol": "PCK2",
  "term_label": "phosphoenolpyruvate carboxykinase (GTP) activity",
  "gene_name": "Phosphoenolpyruvate carboxykinase [GTP], mitochondrial"
}